chloroplast isoamylase complex [GO:0010368] (cellular component) Sources: GOC:tair_curators Relationships: is a type of isoamylase complex [GO:0043033]; is part of chloroplast [GO:0009507] Definition: A protein complex whose composition varies amongst species; in rice it probably exists in a homo-tetramer to homo-hexamer form and in Gram negative bacteria as a dimer. Functions in the hydrolysis of alpha-(1,6)-D-glucosidic branch linkages. Isoamylases in plants are intracellular and probably chloroplast localized.